{
  "gene_name": "Nicotinamide_nicotinic acid mononucleotide adenylyltransferase 1",
  "term_label": "nucleus",
  "gene_symbol": "NMNAT1",
  "term_id": "GO:0005634",
  "gene": "UniProtKB:Q9HAN9"
}